{
  "term_label": "cytosol",
  "term_id": "GO:0005829",
  "gene_symbol": "WDR4",
  "gene_name": "tRNA (guanine-N(7)-)-methyltransferase non-catalytic subunit WDR4",
  "gene": "UniProtKB:P57081"
}